{
  "gene_symbol": "RNF113B",
  "gene": "UniProtKB:Q8IZP6",
  "term_label": "mRNA splicing, via spliceosome",
  "term_id": "GO:0000398",
  "gene_name": "RING finger protein 113B"
}